{
  "gene_symbol": "ALPG",
  "gene": "UniProtKB:P10696",
  "term_id": "GO:0005886",
  "term_label": "plasma membrane",
  "gene_name": "Alkaline phosphatase, germ cell type"
}